{
  "term_label": "ATP binding",
  "gene": "UniProtKB:Q9GZT4",
  "gene_name": "Serine racemase",
  "term_id": "GO:0005524",
  "gene_symbol": "SRR"
}